{
  "term_label": "NAD+ poly-ADP-ribosyltransferase activity",
  "gene_symbol": "PARP16",
  "term_id": "GO:0003950",
  "gene_name": "Protein mono-ADP-ribosyltransferase PARP16",
  "gene": "UniProtKB:Q8N5Y8"
}